negative regulation of glycolytic process [GO:0045820] (biological process) Definition: Any process that stops, prevents, or reduces the frequency, rate or extent of glycolysis. Relationships: is_a GO:0006110; is a type of negative regulation of purine nucleotide catabolic process [GO:0033122]; is a type of negative regulation of carbohydrate metabolic process [GO:0045912]; is a type of GO:1903579; negatively regulates glycolytic process [GO:0006096] Also known as: down regulation of glycolysis, down-regulation of glycolysis, downregulation of glycolysis, inhibition of glycolysis Sources: GOC:go_curators Subtypes: negative regulation of glycolytic process through fructose-6-phosphate [GO:1904539]